RNA binding [GO:0003723] (molecular function) Sources: GOC:jl, GOC:mah Also known as: base pairing with RNA, poly(A) RNA binding, poly(A)-RNA binding, poly-A RNA binding Relationships: is a type of nucleic acid binding [GO:0003676] Subtypes: tRNA binding [GO:0000049], GO:0000339, regulatory region RNA binding [GO:0001069], GO:0002151, double-stranded RNA binding [GO:0003725], GO:0003727, mRNA binding [GO:0003729], 7S RNA binding [GO:0008312], snRNA binding [GO:0017069], GO:0019843, GO:0030515, RNA modification guide activity [GO:0030555], ribonuclease P RNA binding [GO:0033204], GO:0034336, 21U-RNA binding [GO:0034583], RNA stem-loop binding [GO:0035613], pre-mRNA binding [GO:0036002], BRE binding [GO:0042835], telomeric repeat-containing RNA binding [GO:0061752], GO:0061980, pumilio-response element binding [GO:0062104], telomerase RNA binding [GO:0070034], primary miRNA binding [GO:0070878], pre-miRNA binding [GO:0070883], histone pre-mRNA DCP binding [GO:0071208], lncRNA binding [GO:0106222], GO:1904678, GO:1990605 Definition: Binding to an RNA molecule or a portion thereof. Regulation: positively regulated by positive regulation of RNA binding [GO:1905216]